molecular function regulator activity [GO:0098772] (MF) Sources: GOC:dos, GOC:pt Subtypes: G protein activity [GO:0003925], enzyme regulator activity [GO:0030234], GO:0030545, ATPase regulator activity [GO:0060590], molecular sensor activity [GO:0140299], cytoskeletal motor regulator activity [GO:0140659], GO:0140677, molecular function inhibitor activity [GO:0140678], transporter regulator activity [GO:0141108] Definition: A molecular function regulator regulates the activity of its target via non-covalent binding that does not result in covalent modification to the target. Examples of molecular function regulators include regulatory subunits of multimeric enzymes and channels. Mechanisms of regulation include allosteric changes in the target and competitive inhibition. Note: This term should only be used in cases when the regulator directly interacts with the enzyme, but does not result in a covalent modification. Also known as: molecular function regulator Relationships: is a type of molecular_function [GO:0003674]; has part protein binding [GO:0005515]